{
  "gene_symbol": "OR5T3",
  "term_label": "Unknown cellular component",
  "gene_name": "Olfactory receptor 5T3",
  "term_id": "UNKNOWN:0003",
  "gene": "UniProtKB:Q8NGG3"
}